abducens nerve development [GO:0021560] (biological process) Sources: GOC:cls, GOC:dgh, GOC:dph, GOC:jid, GO_REF:0000021 Also known as: cranial nerve 6 development, cranial nerve VI development, CN VI development Definition: The process whose specific outcome is the progression of the abducens nerve over time, from its formation to the mature structure. The motor function of the abducens nerve is to contract the lateral rectus which results in abduction of the eye. Relationships: is_a cranial nerve development [GO:0021545]